{
  "term_id": "GO:0005925",
  "gene_symbol": "TNS4",
  "gene": "UniProtKB:Q8IZW8",
  "term_label": "focal adhesion",
  "gene_name": "Tensin-4"
}